{
  "gene_name": "Homeobox protein cut-like 2",
  "gene": "UniProtKB:O14529",
  "term_label": "RNA polymerase II transcription regulatory region sequence-specific DNA binding",
  "term_id": "GO:0000977",
  "gene_symbol": "CUX2"
}